small ribosomal subunit [GO:0015935] (cellular component) Relationships: is a type of ribosomal subunit [GO:0044391] Sources: GOC:mah Definition: The smaller of the two subunits of a ribosome. Also known as: ribosomal small subunit Subtypes: GO:0000314, cytosolic small ribosomal subunit [GO:0022627]